{
  "gene": "UniProtKB:O75629",
  "gene_symbol": "CREG1",
  "gene_name": "Protein CREG1",
  "term_id": "GO:0005615",
  "term_label": "extracellular space"
}